{
  "term_id": "UNKNOWN:0002",
  "gene_symbol": "CUTA",
  "gene": "UniProtKB:O60888",
  "gene_name": "Protein CutA",
  "term_label": "Unknown biological process"
}